{
  "term_id": "UNKNOWN:0001",
  "gene_symbol": "IGKV1-27",
  "gene_name": "Immunoglobulin kappa variable 1-27",
  "term_label": "Unknown molecular function",
  "gene": "UniProtKB:A0A075B6S5"
}